estradiol 17-beta-dehydrogenase [NAD(P)+] activity [GO:0004303] (molecular function) Relationships: is a type of GO:0033764 Sources: EC:1.1.1.62 Definition: Catalysis of the reaction: estradiol-17-beta + NAD(P)+ = estrone + NAD(P)H + H+. The activity can use NAD+ or NADP+ as the acceptor. Also known as: 17-beta-HSD activity, 17-beta-hydroxysteroid dehydrogenase activity, 20alpha-hydroxysteroid dehydrogenase, 17-beta-estradiol dehydrogenase activity, 17beta,20alpha-hydroxysteroid dehydrogenase activity, 17beta-HSD, 17beta-estradiol dehydrogenase activity, 17beta-hydroxysteroid dehydrogenase activity, estradiol 17-beta-dehydrogenase activity, estradiol 17beta-dehydrogenase activity, estradiol dehydrogenase activity, estradiol-17beta:NAD(P)+ 17-oxidoreductase activity, estrogen 17-oxidoreductase activity